{
  "gene": "UniProtKB:O60831",
  "term_id": "GO:0016020",
  "gene_name": "PRA1 family protein 2",
  "gene_symbol": "PRAF2",
  "term_label": "membrane"
}